{
  "term_id": "UNKNOWN:0001",
  "term_label": "Unknown molecular function",
  "gene_name": "Putative uncharacterized protein encoded by LINC00597",
  "gene_symbol": "LINC00597",
  "gene": "UniProtKB:Q9H2U6"
}